{
  "term_id": "GO:0007188",
  "gene_symbol": "GNA12",
  "gene_name": "Guanine nucleotide-binding protein subunit alpha-12",
  "term_label": "adenylate cyclase-modulating G protein-coupled receptor signaling pathway",
  "gene": "UniProtKB:Q03113"
}